protein deglycation, methylglyoxal removal [GO:0036530] (biological process) Relationships: is a type of methylglyoxal metabolic process [GO:0009438]; is a type of lactate biosynthetic process [GO:0019249]; is a type of protein deglycation [GO:0036525] Definition: The removal of methylglyoxal from a glycated protein, to form lactate and a deglycated protein. References: PMID:25416785 Sources: GOC:PARL, GOC:bf Also known as: protein deglycation of methylglyoxal-glycated protein